{
  "term_id": "GO:0004014",
  "gene_symbol": "AMD1",
  "gene": "UniProtKB:P17707",
  "gene_name": "S-adenosylmethionine decarboxylase proenzyme",
  "term_label": "adenosylmethionine decarboxylase activity"
}